{
  "term_id": "UNKNOWN:0003",
  "term_label": "Unknown cellular component",
  "gene_symbol": "MAP2K2",
  "gene_name": "Dual specificity mitogen-activated protein kinase kinase 2",
  "gene": "UniProtKB:P36507"
}